{
  "term_label": "nucleolus",
  "gene_name": "mRNA turnover protein 4 homolog",
  "gene_symbol": "MRTO4",
  "term_id": "GO:0005730",
  "gene": "UniProtKB:Q9UKD2"
}